{
  "gene_name": "Killer cell immunoglobulin-like receptor 2DL2",
  "term_id": "GO:0002767",
  "gene_symbol": "KIR2DL2",
  "gene": "UniProtKB:P43627",
  "term_label": "immune response-inhibiting cell surface receptor signaling pathway"
}